{
  "gene_name": "Large neutral amino acids transporter small subunit 3",
  "gene": "UniProtKB:O75387",
  "gene_symbol": "SLC43A1",
  "term_id": "GO:0015175",
  "term_label": "neutral L-amino acid transmembrane transporter activity"
}